{
  "term_label": "hippo signaling",
  "gene_symbol": "TEAD3",
  "term_id": "GO:0035329",
  "gene_name": "Transcriptional enhancer factor TEF-5",
  "gene": "UniProtKB:Q99594"
}